{
  "gene_symbol": "SLC12A2",
  "gene": "UniProtKB:P55011",
  "term_id": "GO:0008519",
  "term_label": "ammonium channel activity",
  "gene_name": "Solute carrier family 12 member 2"
}